{
  "gene": "UniProtKB:Q9H832",
  "gene_symbol": "UBE2Z",
  "term_id": "GO:0005634",
  "term_label": "nucleus",
  "gene_name": "Ubiquitin-conjugating enzyme E2 Z"
}